negative regulation of DNA recombination [GO:0045910] (biological process) Sources: GOC:go_curators Relationships: is a type of GO:0000018; is a type of negative regulation of DNA metabolic process [GO:0051053]; negatively regulates DNA recombination [GO:0006310] Subtypes: GO:0007537, negative regulation of reciprocal meiotic recombination [GO:0045128], negative regulation of isotype switching [GO:0045829], negative regulation of mitotic recombination [GO:0045950], negative regulation of DNA recombination at telomere [GO:0048239], GO:0060543, negative regulation of DNA recombination at centromere [GO:0061808], negative regulation of single-strand break repair via homologous recombination [GO:1903111], GO:2000042 Definition: Any process that stops, prevents, or reduces the frequency, rate or extent of DNA recombination. Also known as: down regulation of DNA recombination, down-regulation of DNA recombination, downregulation of DNA recombination, inhibition of DNA recombination